{
  "gene_name": "Arrestin domain-containing protein 5",
  "term_label": "molecular adaptor activity",
  "term_id": "GO:0060090",
  "gene_symbol": "ARRDC5",
  "gene": "UniProtKB:A6NEK1"
}